positive regulation of imaginal disc-derived leg joint morphogenesis [GO:0110138] (biological process) Relationships: is a type of GO:0051094; is a type of GO:0110137; RO_0002213 imaginal disc-derived leg morphogenesis [GO:0007480] Definition: Any process that activates or increases the frequency, rate or extent of imaginal disc-derived leg joint morphogenesis. References: PMID:25329825 Sources: GOC:ha